{
  "term_label": "Unknown cellular component",
  "gene_name": "Protein FAM90A17",
  "gene": "UniProtKB:P0DV74",
  "term_id": "UNKNOWN:0003",
  "gene_symbol": "FAM90A17"
}